{
  "gene": "UniProtKB:P29120",
  "term_id": "GO:0004252",
  "gene_name": "Neuroendocrine convertase 1",
  "term_label": "serine-type endopeptidase activity",
  "gene_symbol": "PCSK1"
}